{
  "gene": "UniProtKB:B1AK53",
  "term_id": "GO:0051015",
  "gene_symbol": "ESPN",
  "gene_name": "Espin",
  "term_label": "actin filament binding"
}